zoospore formation [GO:0075239] (biological process) Definition: The process in which a diploid cell undergoes meiosis, and the meiotic products acquire specialized features of asexual motile mononucleate flagellated spores called zoospores. Sources: GOC:pamgo_curators Regulation: RO_0002211 by GO:0075240; positively regulated by positive regulation of zoospore formation [GO:0075241]; negatively regulated by negative regulation of zoospore formation [GO:0075242] Relationships: is a type of sporangiospore formation [GO:0034300]